{
  "gene_symbol": "MUC5AC",
  "gene": "UniProtKB:P98088",
  "term_label": "extracellular matrix",
  "term_id": "GO:0031012",
  "gene_name": "Mucin-5AC"
}